metallocarboxypeptidase activity [GO:0004181] (molecular function) Relationships: is a type of carboxypeptidase activity [GO:0004180]; is a type of metalloexopeptidase activity [GO:0008235] Definition: Catalysis of the hydrolysis of a single C-terminal amino acid residue from a polypeptide chain by a mechanism in which water acts as a nucleophile, one or two metal ions hold the water molecule in place, and charged amino acid side chains are ligands for the metal ions. Subtypes: zinc D-Ala-D-Ala carboxypeptidase activity [GO:0009046], GO:0061473, GO:0102274, tubulin-tyrosine carboxypeptidase [GO:0106423] Sources: https://www.ebi.ac.uk/merops/about/glossary.shtml#CARBOXYPEPTIDASE